{
  "term_label": "Unknown cellular component",
  "term_id": "UNKNOWN:0003",
  "gene": "UniProtKB:Q8NC74",
  "gene_name": "RBBP8 N-terminal-like protein",
  "gene_symbol": "RBBP8NL"
}